cellular response to ethylene stimulus [GO:0071369] (biological process) Also known as: cellular response to ethene stimulus Definition: Any process that results in a change in state or activity of a cell (in terms of movement, secretion, enzyme production, gene expression, etc.) as a result of an ethylene (ethene) stimulus. Relationships: is a type of response to ethylene [GO:0009723]; is a type of GO:0032870 Sources: GOC:mah